{
  "term_id": "UNKNOWN:0001",
  "gene": "UniProtKB:Q08AG7",
  "gene_name": "Mitotic-spindle organizing protein 1",
  "term_label": "Unknown molecular function",
  "gene_symbol": "MZT1"
}